{
  "term_id": "GO:0005829",
  "gene_name": "Iron-responsive element-binding protein 2",
  "term_label": "cytosol",
  "gene": "UniProtKB:P48200",
  "gene_symbol": "IREB2"
}